{
  "gene_name": "MKI67 FHA domain-interacting nucleolar phosphoprotein",
  "term_id": "GO:0005730",
  "gene_symbol": "NIFK",
  "gene": "UniProtKB:Q9BYG3",
  "term_label": "nucleolus"
}